{
  "gene_symbol": "ZDHHC7",
  "gene": "UniProtKB:Q9NXF8",
  "gene_name": "Palmitoyltransferase ZDHHC7",
  "term_id": "GO:0019706",
  "term_label": "protein-cysteine S-palmitoyltransferase activity"
}